negative regulation of central B cell tolerance induction [GO:0002896] (biological process) Relationships: is a type of GO:0002647; is a type of negative regulation of B cell tolerance induction [GO:0002662]; is a type of GO:0002895; negatively regulates central B cell tolerance induction [GO:0002510] Also known as: down regulation of central B cell tolerance induction, down-regulation of central B cell tolerance induction, downregulation of central B cell tolerance induction, inhibition of central B cell tolerance induction Sources: GOC:add Definition: Any process that stops, prevents, or reduces the frequency, rate, or extent of central B cell tolerance induction. Subtypes: negative regulation of central B cell deletion [GO:0002899], GO:0002915